chaeta morphogenesis [GO:0008407] (biological process) Subtypes: cibarial fish-trap bristle morphogenesis [GO:0048718] Relationships: is a type of animal organ morphogenesis [GO:0009887]; is part of chaeta development [GO:0022416] Also known as: bristle morphogenesis Sources: FBbt:00005177, GOC:bf, GOC:cjm, GOC:dos, GOC:go_curators Definition: The process in which the anatomical structures of the chaeta are generated and organized. A chaeta is a sensory multicellular cuticular outgrowth of a specifically differentiated cell.